{
  "term_id": "GO:0003700",
  "gene_name": "Zinc finger protein 821",
  "gene_symbol": "ZNF821",
  "gene": "UniProtKB:O75541",
  "term_label": "DNA-binding transcription factor activity"
}